{
  "gene_symbol": "SYT10",
  "gene": "UniProtKB:Q6XYQ8",
  "gene_name": "Synaptotagmin-10",
  "term_label": "exocytic vesicle",
  "term_id": "GO:0070382"
}